{
  "gene_symbol": "LINC01590",
  "gene": "UniProtKB:Q5TEZ4",
  "gene_name": "Putative uncharacterized protein encoded by LINC01590",
  "term_id": "UNKNOWN:0002",
  "term_label": "Unknown biological process"
}